interleukin-5-mediated signaling pathway [GO:0038043] (biological process) Relationships: is a type of cytokine-mediated signaling pathway [GO:0019221] Also known as: IL-5-mediated signaling pathway, interleukin-5-mediated signalling pathway Sources: GOC:signaling Definition: The series of molecular signals initiated by interleukin-5 binding to its receptor on the surface of a cell, and ending with the regulation of a downstream cellular process, e.g. transcription.